{
  "gene_symbol": "SHLD3",
  "gene_name": "Shieldin complex subunit 3",
  "term_label": "positive regulation of isotype switching",
  "gene": "UniProtKB:Q6ZNX1",
  "term_id": "GO:0045830"
}